L-serine O-succinyltransferase activity [GO:0160210] (MF) References: PMID:28581482 Sources: RHEA:52820 Definition: Catalysis of the reaction: L-serine + succinyl-CoA = CoA + O-succinyl-L-serine. Relationships: is a type of GO:0016750